Methanosarcina-phenazine hydrogenase activity [GO:0051911] (molecular function) Sources: EC:1.12.98.3 Also known as: methanophenazine hydrogenase activity, methylviologen-reducing hydrogenase activity, coenzyme-M-7-mercaptoheptanoylthreonine-phosphate-heterodisulfide hydrogenase activity, hydrogen:2-(2,3-dihydropentaprenyloxy)phenazine oxidoreductase activity Definition: Catalysis of the reaction: H2 + 2-(2,3-dihydropentaprenyloxy)phenazine = 2-dihydropentaprenyloxyphenazine. Relationships: is a type of oxidoreductase activity, acting on hydrogen as donor, with other known acceptors [GO:0046995]